T-helper cell lineage commitment [GO:0002295] (biological process) Definition: The process in which a CD4-positive, alpha-beta T cell becomes committed to becoming a T-helper cell, a CD4-positive, alpha-beta T cell specialized to promote various immunological processes. Also known as: T-helper cell fate commitment, Th0 lineage commitment, Thp lineage commitment Subtypes: GO:0002296, T-helper 2 cell lineage commitment [GO:0002297], T-helper 17 cell lineage commitment [GO:0072540] Relationships: is a type of CD4-positive, alpha-beta T cell lineage commitment [GO:0043373]; is part of T-helper cell differentiation [GO:0042093] Sources: GOC:add, ISBN:0781735149